{
  "gene_symbol": "CATSPERE",
  "term_label": "flagellated sperm motility",
  "term_id": "GO:0030317",
  "gene_name": "Cation channel sperm-associated auxiliary subunit epsilon",
  "gene": "UniProtKB:Q5SY80"
}